{
  "gene_name": "Intersectin-2",
  "term_id": "GO:0030674",
  "gene_symbol": "ITSN2",
  "gene": "UniProtKB:Q9NZM3",
  "term_label": "protein-macromolecule adaptor activity"
}